{
  "gene_name": "Keratin, type I cytoskeletal 27",
  "gene": "UniProtKB:Q7Z3Y8",
  "gene_symbol": "KRT27",
  "term_id": "GO:0005856",
  "term_label": "cytoskeleton"
}